negative regulation of neuromuscular junction development [GO:1904397] (BP) References: PMID:7722643 Sources: GOC:TermGenie, GO_REF:0000058 Also known as: down regulation of neuromuscular junction development, down regulation of neuromuscular junction organization, down-regulation of neuromuscular junction development, down-regulation of neuromuscular junction organization, downregulation of neuromuscular junction development, downregulation of neuromuscular junction organization, negative regulation of neuromuscular junction organization, inhibition of neuromuscular junction development, inhibition of neuromuscular junction organization, down regulation of NMJ stability, down regulation of neuromuscular junction stability, down-regulation of NMJ stability, down-regulation of neuromuscular junction stability, downregulation of NMJ stability, downregulation of neuromuscular junction stability, inhibition of NMJ stability, inhibition of neuromuscular junction stability, negative regulation of NMJ stability, negative regulation of neuromuscular junction stability Definition: Any process that stops, prevents or reduces the frequency, rate or extent of neuromuscular junction development. Subtypes: negative regulation of synaptic assembly at neuromuscular junction [GO:0045886] Relationships: is a type of GO:1904396; is a type of negative regulation of synapse organization [GO:1905809]; negatively regulates neuromuscular junction development [GO:0007528]